maintenance of unfolded protein involved in ERAD pathway [GO:1904378] (biological process) Definition: Maintaining an endoplasmic reticulum (ER) protein in an unfolded, soluble state that contributes to its degradation by the cytoplasmic proteasome. Maintaining ER-resident proteins in an unfolded yet soluble state condition after their retro-translocation favors their turnover by the cytosolic proteasome. Also known as: maintenance of unfolded protein involved in endoplasmic reticulum-associated degradation, ERAD chaperone-like activity, chaperone holdase activity, holdase activity, maintenance of unfolded protein during ERAD, maintenance of unfolded protein involved in ER-associated degradation pathway, maintenance of unfolded protein involved in endoplasmic reticulum-associated protein degradation pathway References: PMID:21636303 Sources: GOC:BHF, GOC:PARL, GOC:TermGenie, GOC:bf, GOC:nc Relationships: is a type of maintenance of unfolded protein [GO:0036506]; is part of ERAD pathway [GO:0036503]